{
  "gene_name": "Semaphorin-4A",
  "term_id": "GO:0001755",
  "gene_symbol": "SEMA4A",
  "gene": "UniProtKB:Q9H3S1",
  "term_label": "neural crest cell migration"
}